{
  "gene": "UniProtKB:Q8NH95",
  "gene_name": "Putative olfactory receptor 13C6",
  "gene_symbol": "OR13C6P",
  "term_id": "GO:0050911",
  "term_label": "detection of chemical stimulus involved in sensory perception of smell"
}